{
  "term_label": "glutamatergic synapse",
  "gene": "UniProtKB:Q13574",
  "term_id": "GO:0098978",
  "gene_name": "Diacylglycerol kinase zeta",
  "gene_symbol": "DGKZ"
}